{
  "gene": "UniProtKB:Q03169",
  "term_label": "exocyst localization",
  "term_id": "GO:0051601",
  "gene_name": "Tumor necrosis factor alpha-induced protein 2",
  "gene_symbol": "TNFAIP2"
}